{
  "term_id": "UNKNOWN:0003",
  "gene": "UniProtKB:Q8NEF3",
  "gene_symbol": "CCDC112",
  "gene_name": "Coiled-coil domain-containing protein 112",
  "term_label": "Unknown cellular component"
}